{
  "gene": "UniProtKB:Q5JUX0",
  "gene_name": "Spindlin-3",
  "term_id": "GO:0006355",
  "gene_symbol": "SPIN3",
  "term_label": "regulation of DNA-templated transcription"
}